{
  "term_id": "GO:0099577",
  "gene": "UniProtKB:Q06787",
  "gene_name": "Fragile X messenger ribonucleoprotein 1",
  "gene_symbol": "FMR1",
  "term_label": "regulation of translation at presynapse, modulating synaptic transmission"
}